{
  "term_id": "UNKNOWN:0002",
  "gene_name": "NmrA-like family domain-containing protein 1",
  "term_label": "Unknown biological process",
  "gene_symbol": "NMRAL1",
  "gene": "UniProtKB:Q9HBL8"
}